{
  "gene_name": "Collectin-10",
  "gene": "UniProtKB:Q9Y6Z7",
  "term_id": "UNKNOWN:0001",
  "term_label": "Unknown molecular function",
  "gene_symbol": "COLEC10"
}